{
  "gene_symbol": "C3orf84",
  "gene_name": "Uncharacterized protein C3orf84",
  "term_id": "UNKNOWN:0002",
  "term_label": "Unknown biological process",
  "gene": "UniProtKB:H3BNL1"
}